oxytocin receptor activity [GO:0004990] (molecular function) Sources: GOC:ai Relationships: is a type of G protein-coupled peptide receptor activity [GO:0008528] Definition: Combining with oxytocin to initiate a change in cell activity.